{
  "gene_symbol": "ATG9A",
  "term_id": "GO:0005776",
  "gene": "UniProtKB:Q7Z3C6",
  "term_label": "autophagosome",
  "gene_name": "Autophagy-related protein 9A"
}